{
  "gene_symbol": "POLR1C",
  "term_label": "RNA polymerase I complex",
  "term_id": "GO:0005736",
  "gene_name": "DNA-directed RNA polymerases I and III subunit RPAC1",
  "gene": "UniProtKB:O15160"
}